maturation of 5.8S rRNA from tricistronic rRNA transcript (SSU-rRNA, 5.8S rRNA, LSU-rRNA) [GO:0000466] (biological process) References: PMID:10690410 Sources: GOC:curators Definition: Any process involved in the maturation of an rRNA molecule originally produced as part of a tricistronic rRNA transcript that contained the Small SubUnit (SSU) rRNA, the 5.8S rRNA, and the Large SubUnit (LSU) rRNA, in that order, from 5' to 3' along the primary transcript. Relationships: is_a maturation of 5.8S rRNA [GO:0000460]